cell migration involved in kidney development [GO:0035787] (biological process) Sources: GOC:bf, GOC:mtg_kidney_jan10, GOC:yaf Subtypes: cell migration involved in metanephros development [GO:0035788], mesenchymal stem cell migration involved in uteric bud morphogenesis [GO:0061456], GO:0072155 Definition: The orderly movement of a cell from one site to another that will contribute to the progression of the kidney over time, from its formation to the mature organ. Relationships: is a type of cell migration [GO:0016477]; is part of GO:0001822